inositol pentakisphosphate kinase activity [GO:0120517] (molecular function) Sources: GOC:curators Subtypes: inositol-1,3,4,5,6-pentakisphosphate 2-kinase activity [GO:0035299], GO:0102732 Relationships: is a type of phosphotransferase activity, alcohol group as acceptor [GO:0016773]; is a type of inositol phosphate kinase activity [GO:0180030] Definition: Catalysis of the reaction: inositol pentakisphosphate + ATP = inositol hexakisphosphate + ADP + H+.